connective tissue replacement involved in inflammatory response wound healing [GO:0002248] (biological process) Regulation: regulated by regulation of connective tissue replacement involved in inflammatory response wound healing [GO:1904596]; negatively regulated by negative regulation of connective tissue replacement involved in inflammatory response wound healing [GO:1904597]; positively regulated by positive regulation of connective tissue replacement involved in inflammatory response wound healing [GO:1904598] Relationships: is a type of connective tissue replacement [GO:0097709]; is part of wound healing involved in inflammatory response [GO:0002246] Also known as: fibrosis during inflammatory response, tissue fibrosis development, connective tissue replacement during inflammatory response References: PMID:9639571 Sources: GOC:jal Definition: The series of events leading to growth of connective tissue when loss of tissues that are incapable of regeneration occurs, or when fibrinous exudate cannot be adequately cleared, as part of an inflammatory response.